positive regulation of mRNA binding [GO:1902416] (biological process) Definition: Any process that activates or increases the frequency, rate or extent of mRNA binding. Also known as: up regulation of mRNA binding, up-regulation of mRNA binding, upregulation of mRNA binding, activation of mRNA binding Relationships: is a type of regulation of mRNA binding [GO:1902415]; is a type of positive regulation of RNA binding [GO:1905216]; positively regulates mRNA binding [GO:0003729] References: PMID:22890846 Sources: GOC:TermGenie, GOC:rb